regulation of protein localization to nucleolus [GO:1904749] (biological process) References: PMID:24415760 Sources: GOC:BHF, GOC:BHF_telomere, GOC:TermGenie, GOC:nc, GO_REF:0000058 Relationships: is a type of regulation of protein localization to nucleus [GO:1900180]; regulates protein localization to nucleolus [GO:1902570] Subtypes: negative regulation of protein localization to nucleolus [GO:1904750], positive regulation of protein localization to nucleolus [GO:1904751] Definition: Any process that modulates the frequency, rate or extent of protein localization to nucleolus. Also known as: regulation of protein localisation in nucleolus, regulation of protein localisation to nucleolus, regulation of protein localization in nucleolus